{
  "term_id": "GO:0000976",
  "gene_symbol": "BAHD1",
  "gene_name": "Bromo adjacent homology domain-containing 1 protein",
  "gene": "UniProtKB:Q8TBE0",
  "term_label": "transcription cis-regulatory region binding"
}